{
  "gene": "UniProtKB:Q32P51",
  "gene_symbol": "HNRNPA1L2",
  "gene_name": "Heterogeneous nuclear ribonucleoprotein A1-like 2",
  "term_label": "mRNA splicing, via spliceosome",
  "term_id": "GO:0000398"
}